gamma-delta T cell proliferation involved in immune response [GO:0002311] (BP) Definition: The expansion of a gamma-delta T cell population by cell division as part of an immune response. Sources: GOC:add Relationships: is a type of gamma-delta T cell activation involved in immune response [GO:0002290]; is_a T cell proliferation involved in immune response [GO:0002309]; is a type of gamma-delta T cell proliferation [GO:0046630] Also known as: gamma-delta T cell proliferation during immune response, gamma-delta T lymphocyte proliferation during immune response, gamma-delta T-cell proliferation during immune response, gamma-delta T-lymphocyte proliferation during immune response